{
  "gene": "UniProtKB:Q30KQ5",
  "gene_symbol": "DEFB115",
  "gene_name": "Beta-defensin 115",
  "term_id": "UNKNOWN:0003",
  "term_label": "Unknown cellular component"
}